{
  "gene": "UniProtKB:Q3KQV3",
  "term_id": "GO:0000981",
  "term_label": "DNA-binding transcription factor activity, RNA polymerase II-specific",
  "gene_name": "Zinc finger protein 792",
  "gene_symbol": "ZNF792"
}